SA node cell action potential [GO:0086015] (biological process) Regulation: RO_0002211 by regulation of SA node cell action potential [GO:0098907] Also known as: SA node cardiac muscle cell action potential, SAN cardiac muscle cell action potential, sinoatrial node cardiac muscle cell action potential, sinus node cardiac muscle cell action potential Relationships: is a type of cardiac muscle cell action potential [GO:0086001]; is part of SA node cell to atrial cardiac muscle cell signaling [GO:0086018] Definition: An action potential that occurs in a sinoatrial node cardiac muscle cell. Sources: GOC:BHF, GOC:mtg_cardiac_conduct_nov11